xyloglucan 1,6-alpha-xylosidase activity [GO:0080176] (molecular function) Definition: Catalysis of the hydrolysis of xyloglucan side chains so as to remove unsubstituted D-xylose residues attached to the glucose located at the non-reducing terminus. References: PMID:20801759 Relationships: is a type of hydrolase activity, hydrolyzing O-glycosyl compounds [GO:0004553]